{
  "term_id": "GO:0030036",
  "term_label": "actin cytoskeleton organization",
  "gene_symbol": "SPTAN1",
  "gene_name": "Spectrin alpha chain, non-erythrocytic 1",
  "gene": "UniProtKB:Q13813"
}